{
  "gene_symbol": "IL24",
  "gene": "UniProtKB:Q13007",
  "term_id": "GO:0005125",
  "gene_name": "Interleukin-24",
  "term_label": "cytokine activity"
}